negative regulation of circadian sleep/wake cycle, REM sleep [GO:0042322] (biological process) Sources: GOC:go_curators, GOC:jl Also known as: down regulation of circadian sleep/wake cycle, REM sleep, down-regulation of circadian sleep/wake cycle, REM sleep, downregulation of circadian sleep/wake cycle, REM sleep, negative regulation of REM sleep, inhibition of circadian sleep/wake cycle, REM sleep Definition: Any process that stops, prevents or reduces the duration or quality of rapid eye movement (REM) sleep. Relationships: is a type of regulation of circadian sleep/wake cycle, REM sleep [GO:0042320]; is a type of negative regulation of circadian sleep/wake cycle, sleep [GO:0042321]; negatively regulates circadian sleep/wake cycle, REM sleep [GO:0042747]